{
  "term_id": "GO:0005858",
  "gene_name": "Dynein axonemal heavy chain 12",
  "gene_symbol": "DNAH12",
  "gene": "UniProtKB:Q6ZR08",
  "term_label": "axonemal dynein complex"
}